{
  "term_id": "UNKNOWN:0002",
  "term_label": "Unknown biological process",
  "gene": "UniProtKB:Q8WZ82",
  "gene_name": "Esterase OVCA2",
  "gene_symbol": "OVCA2"
}